{
  "term_label": "nucleus",
  "gene_symbol": "RBM7",
  "gene_name": "RNA-binding protein 7",
  "term_id": "GO:0005634",
  "gene": "UniProtKB:Q9Y580"
}